{
  "gene": "UniProtKB:P68032",
  "term_label": "sarcomere",
  "gene_name": "Actin, alpha cardiac muscle 1",
  "gene_symbol": "ACTC1",
  "term_id": "GO:0030017"
}